{
  "gene_symbol": "B3GALT2",
  "gene": "UniProtKB:O43825",
  "term_label": "Golgi membrane",
  "term_id": "GO:0000139",
  "gene_name": "Beta-1,3-galactosyltransferase 2"
}